{
  "term_id": "UNKNOWN:0003",
  "term_label": "Unknown cellular component",
  "gene_name": "Immunoglobulin heavy variable 3-23",
  "gene": "UniProtKB:P01764",
  "gene_symbol": "IGHV3-23"
}